{
  "gene": "UniProtKB:Q5VV41",
  "term_id": "UNKNOWN:0003",
  "term_label": "Unknown cellular component",
  "gene_name": "Rho guanine nucleotide exchange factor 16",
  "gene_symbol": "ARHGEF16"
}